{
  "gene_name": "Keratin, type II cuticular Hb3",
  "term_id": "GO:0045095",
  "gene": "UniProtKB:P78385",
  "gene_symbol": "KRT83",
  "term_label": "keratin filament"
}